{
  "term_label": "GTP binding",
  "gene": "UniProtKB:Q13885",
  "gene_name": "Tubulin beta-2A chain",
  "term_id": "GO:0005525",
  "gene_symbol": "TUBB2A"
}